{
  "term_id": "GO:0005634",
  "term_label": "nucleus",
  "gene": "UniProtKB:Q6ZN32",
  "gene_name": "ETS translocation variant 3-like protein",
  "gene_symbol": "ETV3L"
}